regulation of cardiac muscle cell action potential involved in regulation of contraction [GO:0098909] (biological process) Sources: GOC:BHF, GOC:mtg_cardiac_conduct_nov11 Definition: Any process that modulates the frequency, rate or extent of action potential creation, propagation or termination in a cardiac muscle cell contributing to the regulation of its contraction. Relationships: is a type of regulation of cardiac muscle cell action potential [GO:0098901]; is part of GO:0086004